{
  "gene": "UniProtKB:O14979",
  "gene_name": "Heterogeneous nuclear ribonucleoprotein D-like",
  "term_label": "RNA binding",
  "term_id": "GO:0003723",
  "gene_symbol": "HNRNPDL"
}